{
  "term_label": "extracellular space",
  "term_id": "GO:0005615",
  "gene_symbol": "DEFA4",
  "gene_name": "Defensin alpha 4",
  "gene": "UniProtKB:P12838"
}